palmitic acid catabolic process [GO:1900534] (biological process) Definition: The chemical reactions and pathways resulting in the breakdown of palmitic acid. Sources: GOC:TermGenie Relationships: is a type of long-chain fatty acid catabolic process [GO:0042758] Regulation: regulated by regulation of palmitic acid catabolic process [GO:0106393]; negatively regulated by negative regulation of palmitic acid catabolic process [GO:0106394]; RO_0002213 by GO:0106395